{
  "term_id": "GO:0030425",
  "gene": "UniProtKB:Q7L099",
  "term_label": "dendrite",
  "gene_name": "Protein RUFY3",
  "gene_symbol": "RUFY3"
}